{
  "gene": "UniProtKB:Q9NWX5",
  "term_id": "UNKNOWN:0002",
  "gene_symbol": "ASB6",
  "gene_name": "Ankyrin repeat and SOCS box protein 6",
  "term_label": "Unknown biological process"
}